{
  "gene_symbol": "DAB2",
  "term_label": "positive regulation of endocytosis",
  "gene_name": "Disabled homolog 2",
  "term_id": "GO:0045807",
  "gene": "UniProtKB:P98082"
}